{
  "term_id": "UNKNOWN:0002",
  "gene": "UniProtKB:Q8N1I8",
  "gene_name": "Putative uncharacterized protein encoded by CACTIN-AS1",
  "term_label": "Unknown biological process",
  "gene_symbol": "CACTIN-AS1"
}